{
  "gene_symbol": "GCK",
  "gene_name": "Hexokinase-4",
  "term_id": "GO:0004340",
  "gene": "UniProtKB:P35557",
  "term_label": "glucokinase activity"
}